{
  "gene": "UniProtKB:P98161",
  "term_label": "monoatomic cation channel activity",
  "gene_name": "Polycystin-1",
  "term_id": "GO:0005261",
  "gene_symbol": "PKD1"
}